JUN kinase binding [GO:0008432] (molecular function) Sources: GOC:jl Relationships: is a type of protein kinase binding [GO:0019901] Definition: Binding to JUN kinase, an enzyme that catalyzes the phosphorylation and activation of members of the JUN family. Also known as: JNK binding